{
  "gene": "UniProtKB:P09669",
  "term_id": "UNKNOWN:0002",
  "term_label": "Unknown biological process",
  "gene_name": "Cytochrome c oxidase subunit 6C",
  "gene_symbol": "COX6C"
}